{
  "gene": "UniProtKB:Q5K131",
  "term_id": "UNKNOWN:0001",
  "term_label": "Unknown molecular function",
  "gene_name": "Chronic lymphocytic leukemia up-regulated protein 1",
  "gene_symbol": "CLLU1"
}